{
  "term_label": "purine nucleobase metabolic process",
  "term_id": "GO:0006144",
  "gene": "UniProtKB:P02766",
  "gene_name": "Transthyretin",
  "gene_symbol": "TTR"
}